{
  "gene_symbol": "FNBP1L",
  "gene_name": "Formin-binding protein 1-like",
  "term_id": "UNKNOWN:0003",
  "term_label": "Unknown cellular component",
  "gene": "UniProtKB:Q5T0N5"
}